{
  "term_label": "olfactory receptor activity",
  "term_id": "GO:0004984",
  "gene_symbol": "OR14I1",
  "gene": "UniProtKB:A6ND48",
  "gene_name": "Olfactory receptor 14I1"
}